{
  "gene": "UniProtKB:P28335",
  "term_id": "GO:0005886",
  "gene_symbol": "HTR2C",
  "gene_name": "5-hydroxytryptamine receptor 2C",
  "term_label": "plasma membrane"
}